UDPG:cyclo-DOPA 5-O-glucosyltransferase activity [GO:0102894] (molecular function) References: PMID:15196939, PMID:15695438 Sources: GOC:pz Relationships: is a type of hexosyltransferase activity [GO:0016758] Definition: Catalysis of the reaction: UDP-alpha-D-glucose + leucodopachrome = H+ + cyclo-dopa 5-O-glucoside + UDP.